{
  "term_label": "regulation of exit from mitosis",
  "term_id": "GO:0007096",
  "gene_name": "Dual specificity protein phosphatase CDC14B",
  "gene_symbol": "CDC14B",
  "gene": "UniProtKB:O60729"
}